lateral part of motile cell [GO:0031255] (cellular component) Definition: The area of a motile cell perpendicular to the direction of movement. Relationships: is a type of lateral part of cell [GO:0097574] Sources: GOC:pg, GOC:pr